{
  "gene_name": "Inhibitor of growth protein 5",
  "term_id": "GO:0003682",
  "gene_symbol": "ING5",
  "term_label": "chromatin binding",
  "gene": "UniProtKB:Q8WYH8"
}